{
  "gene_name": "Lipase maturation factor 2",
  "term_id": "GO:0051604",
  "term_label": "protein maturation",
  "gene_symbol": "LMF2",
  "gene": "UniProtKB:Q9BU23"
}